{
  "gene_name": "Leucine-rich repeat neuronal protein 4",
  "term_label": "plasma membrane",
  "term_id": "GO:0005886",
  "gene": "UniProtKB:Q8WUT4",
  "gene_symbol": "LRRN4"
}